histone deacetylase regulator activity [GO:0035033] (molecular function) Sources: GOC:bf Note: See also the molecular function term 'histone deacetylase activity ; GO:0004407'. Relationships: is a type of enzyme regulator activity [GO:0030234]; has part GO:0042826; regulates histone deacetylase activity [GO:0004407] Subtypes: histone deacetylase inhibitor activity [GO:0046811] Definition: Binds to and modulates the activity of histone deacetylase.